bicarbonate transport [GO:0015701] (biological process) Relationships: is a type of organic anion transport [GO:0015711] Definition: The directed movement of bicarbonate into, out of or within a cell, or between cells, by means of some agent such as a transporter or pore. Sources: GOC:krc Also known as: hydrogencarbonate transport